{
  "gene_name": "Death domain-containing protein CRADD",
  "term_id": "GO:0030330",
  "gene": "UniProtKB:P78560",
  "gene_symbol": "CRADD",
  "term_label": "DNA damage response, signal transduction by p53 class mediator"
}